{
  "gene_symbol": "IKZF4",
  "gene_name": "Zinc finger protein Eos",
  "term_label": "RNA polymerase II cis-regulatory region sequence-specific DNA binding",
  "gene": "UniProtKB:Q9H2S9",
  "term_id": "GO:0000978"
}